{
  "gene_symbol": "SDCCAG8",
  "gene_name": "Serologically defined colon cancer antigen 8",
  "term_id": "GO:0030010",
  "term_label": "establishment of cell polarity",
  "gene": "UniProtKB:Q86SQ7"
}